{
  "gene_name": "ATP-binding cassette sub-family B member 10, mitochondrial",
  "term_id": "UNKNOWN:0001",
  "gene_symbol": "ABCB10",
  "term_label": "Unknown molecular function",
  "gene": "UniProtKB:Q9NRK6"
}